positive regulation of stomatal complex development [GO:2000123] (BP) Sources: GOC:obol Relationships: is a type of positive regulation of post-embryonic development [GO:0048582]; is a type of regulation of stomatal complex development [GO:2000038]; positively regulates stomatal complex development [GO:0010374] Definition: Any process that activates or increases the frequency, rate or extent of stomatal complex development.